positive regulation of axon extension involved in regeneration [GO:0048691] (biological process) Sources: GOC:dgh, GOC:dph, GOC:jid, GOC:lm Also known as: up regulation of axon extension involved in regeneration, up-regulation of axon extension involved in regeneration, upregulation of axon extension involved in regeneration, activation of axon extension involved in regeneration, stimulation of axon extension involved in regeneration Relationships: is a type of positive regulation of axon extension [GO:0045773]; is a type of GO:0048687; is a type of regulation of axon extension involved in regeneration [GO:0048690]; positively regulates axon extension involved in regeneration [GO:0048677] Definition: Any process that activates, maintains or increases the rate of axon extension involved in regeneration.